{
  "gene_name": "Immunoglobulin lambda constant 3",
  "term_label": "IgG immunoglobulin complex",
  "gene_symbol": "IGLC3",
  "term_id": "GO:0071735",
  "gene": "UniProtKB:P0DOY3"
}